{
  "gene_symbol": "ELOVL1",
  "term_id": "GO:0034625",
  "gene": "UniProtKB:Q9BW60",
  "term_label": "fatty acid elongation, monounsaturated fatty acid",
  "gene_name": "Elongation of very long chain fatty acids protein 1"
}